{
  "gene_symbol": "SLAIN2",
  "term_label": "positive regulation of microtubule polymerization",
  "gene": "UniProtKB:Q9P270",
  "term_id": "GO:0031116",
  "gene_name": "SLAIN motif-containing protein 2"
}